{
  "term_id": "GO:0043124",
  "term_label": "negative regulation of canonical NF-kappaB signal transduction",
  "gene_name": "Tumor necrosis factor alpha-induced protein 3",
  "gene_symbol": "TNFAIP3",
  "gene": "UniProtKB:P21580"
}